{
  "term_label": "synapse assembly",
  "gene": "UniProtKB:Q8N0Z9",
  "term_id": "GO:0007416",
  "gene_name": "V-set and immunoglobulin domain-containing protein 10",
  "gene_symbol": "VSIG10"
}